benomyl:proton antiporter activity [GO:0015310] (MF) Definition: Enables the transfer of a solute or solutes from one side of a membrane to the other according to the reaction: H+(out) + benomyl(in) = H+(in) + benomyl(out). Relationships: is a type of GO:0015078; is a type of antiporter activity [GO:0015297]; is a type of GO:0042887 Sources: TC:2.A.1.2.6 Also known as: benomyl:hydrogen antiporter activity